{
  "gene_symbol": "SARM1",
  "term_id": "GO:0030425",
  "gene": "UniProtKB:Q6SZW1",
  "gene_name": "NAD(+) hydrolase SARM1",
  "term_label": "dendrite"
}